{
  "gene_symbol": "KCNK18",
  "gene_name": "Potassium channel subfamily K member 18",
  "term_id": "GO:0022841",
  "term_label": "potassium ion leak channel activity",
  "gene": "UniProtKB:Q7Z418"
}